positive regulation of oxidoreductase activity [GO:0051353] (biological process) Definition: Any process that activates or increases the frequency, rate or extent of oxidoreductase activity, the catalysis of an oxidation-reduction (redox) reaction, a reversible chemical reaction in which the oxidation state of an atom or atoms within a molecule is altered. Sources: GOC:ai Subtypes: positive regulation of NAD(P)H oxidase activity [GO:0033864], positive regulation of nitric-oxide synthase activity [GO:0051000], positive regulation of superoxide dismutase activity [GO:1901671], positive regulation of catalase activity [GO:1902553], positive regulation of succinate dehydrogenase activity [GO:1904231] Also known as: oxidoreductase activator, up regulation of oxidoreductase activity, up-regulation of oxidoreductase activity, upregulation of oxidoreductase activity, activation of oxidoreductase activity, ribonucleotide reductase activating enzyme activity, stimulation of oxidoreductase activity Relationships: is a type of positive regulation of catalytic activity [GO:0043085]; is a type of GO:0051341; positively regulates GO:0016491